{
  "gene_symbol": "ZNF133",
  "gene_name": "Zinc finger protein 133",
  "term_label": "regulation of transcription by RNA polymerase II",
  "gene": "UniProtKB:P52736",
  "term_id": "GO:0006357"
}